{
  "gene_name": "T cell receptor beta variable 12-5",
  "gene_symbol": "TRBV12-5",
  "term_id": "GO:0005886",
  "term_label": "plasma membrane",
  "gene": "UniProtKB:A0A1B0GX78"
}